{
  "gene_name": "Brain acid soluble protein 1",
  "gene": "UniProtKB:P80723",
  "term_label": "cytoplasm",
  "gene_symbol": "BASP1",
  "term_id": "GO:0005737"
}